{
  "term_id": "GO:0005886",
  "gene_name": "Potassium voltage-gated channel subfamily H member 8",
  "term_label": "plasma membrane",
  "gene": "UniProtKB:Q96L42",
  "gene_symbol": "KCNH8"
}